{
  "term_label": "apical plasma membrane",
  "gene_name": "Placenta-expressed transcript 1 protein",
  "term_id": "GO:0016324",
  "gene": "UniProtKB:Q6UQ28",
  "gene_symbol": "PLET1"
}